{
  "gene_symbol": "LEP",
  "term_label": "response to insulin",
  "gene_name": "Leptin",
  "gene": "UniProtKB:P41159",
  "term_id": "GO:0032868"
}